{
  "gene_symbol": "ULK2",
  "term_label": "mitophagy",
  "gene_name": "Serine_threonine-protein kinase ULK2",
  "term_id": "GO:0000423",
  "gene": "UniProtKB:Q8IYT8"
}